{
  "gene": "UniProtKB:O75298",
  "gene_symbol": "RTN2",
  "gene_name": "Reticulon-2",
  "term_label": "neuron differentiation",
  "term_id": "GO:0030182"
}